negative regulation of odontoblast differentiation [GO:1901330] (BP) Sources: GOC:TermGenie Relationships: is a type of inhibition of neuroepithelial cell differentiation [GO:0002085]; is a type of regulation of odontoblast differentiation [GO:1901329]; negatively regulates GO:0071895 Definition: Any process that stops, prevents or reduces the frequency, rate or extent of odontoblast differentiation. Also known as: down regulation of odontoblast differentiation, down-regulation of odontoblast differentiation, downregulation of odontoblast differentiation, inhibition of odontoblast differentiation